poly-N-acetyllactosamine catabolic process [GO:0030310] (biological process) Also known as: poly-N-acetyllactosamine breakdown, poly-N-acetyllactosamine catabolism, poly-N-acetyllactosamine degradation References: PMID:9405606 Sources: GOC:mah Relationships: is a type of aminoglycan catabolic process [GO:0006026]; is a type of poly-N-acetyllactosamine metabolic process [GO:0030309] Definition: The chemical reactions and pathways resulting in the breakdown of poly-N-acetyllactosamine, a carbohydrate composed of N-acetyllactosamine repeats (Gal-beta-1,4-GlcNAc-beta-1,3)n.